ciliary transition fiber assembly [GO:1905353] (BP) References: PMID:24189274 Sources: GOC:TermGenie, GOC:cilia, GO_REF:0000079 Definition: The aggregation, arrangement and bonding together of a set of components to form a ciliary transition fiber. Also known as: cilial transition fiber assembly, cilial transition fiber formation, cilial transition fibre assembly, cilial transition fibre formation, ciliary transition fiber formation, ciliary transition fibre assembly, ciliary transition fibre formation, cilium transition fiber assembly, cilium transition fiber formation, cilium transition fibre assembly, cilium transition fibre formation, centriolar distal appendage assembly, centriolar distal appendage formation, distal appendage of basal body assembly, distal appendage of basal body formation, distal appendage of centriole assembly, distal appendage of centriole formation, distal appendage of mother centriole assembly, distal appendage of mother centriole formation Relationships: is a type of protein-containing complex assembly [GO:0065003]